cellotetraose binding [GO:0044586] (molecular function) Sources: GOC:mengo_curators, GOC:tt Relationships: is a type of GO:0070492 Definition: Binding to a cellotetraose, an oligosaccharide consisting of four glucose residues resulting from hydrolysis of cellulose.